{
  "term_id": "GO:0030854",
  "gene_name": "Calcineurin B homologous protein 3",
  "gene": "UniProtKB:Q96BS2",
  "gene_symbol": "TESC",
  "term_label": "positive regulation of granulocyte differentiation"
}